regulation of sodium ion transmembrane transporter activity [GO:2000649] (biological process) Subtypes: regulation of P-type sodium:potassium-exchanging transporter activity [GO:1903406], regulation of voltage-gated sodium channel activity [GO:1905150], positive regulation of sodium ion transmembrane transporter activity [GO:2000651] Sources: GOC:obol Relationships: is a type of regulation of transmembrane transporter activity [GO:0022898]; is a type of regulation of sodium ion transmembrane transport [GO:1902305]; regulates sodium ion transmembrane transporter activity [GO:0015081] Definition: Any process that modulates the frequency, rate or extent of sodium ion transmembrane transporter activity. Also known as: regulation of sodium transporter activity